{
  "gene_symbol": "RPL41",
  "gene": "UniProtKB:P62945",
  "term_id": "GO:0002181",
  "term_label": "cytoplasmic translation",
  "gene_name": "Large ribosomal subunit protein eL41"
}